phosphate transmembrane transporter activity [GO:0005315] (molecular function) Definition: Enables the transfer of phosphate ions from one side of a membrane to the other, up its concentration gradient. The transporter binds the solute and undergoes a series of conformational changes. Transport works equally well in either direction and is driven by a chemiosmotic source of energy. Secondary active transporters include symporters and antiporters. Also known as: inorganic phosphate transmembrane transporter activity Subtypes: sodium:phosphate symporter activity [GO:0005436], GO:0009673, GO:0015315, dicarboxylate:phosphate antiporter activity [GO:0015364], ATPase-coupled phosphate ion transmembrane transporter activity [GO:0015415], GO:0048249, phosphate ion uniporter activity [GO:0140787] Sources: GOC:mtg_transport Relationships: is a type of secondary active transmembrane transporter activity [GO:0015291]